{
  "gene_symbol": "C16orf82",
  "term_label": "Unknown cellular component",
  "term_id": "UNKNOWN:0003",
  "gene": "UniProtKB:Q7Z2V1",
  "gene_name": "Protein TNT"
}